{
  "gene_name": "Signal transducer and activator of transcription 3",
  "gene": "UniProtKB:P40763",
  "term_label": "response to peptide hormone",
  "term_id": "GO:0043434",
  "gene_symbol": "STAT3"
}